{
  "gene_name": "Interleukin-2 receptor subunit beta",
  "gene_symbol": "IL2RB",
  "gene": "UniProtKB:P14784",
  "term_id": "GO:0016064",
  "term_label": "immunoglobulin mediated immune response"
}